{
  "gene_name": "Interleukin-5",
  "term_label": "extracellular region",
  "gene": "UniProtKB:P05113",
  "term_id": "GO:0005576",
  "gene_symbol": "IL5"
}